{
  "gene_symbol": "ENPP1",
  "gene": "UniProtKB:P22413",
  "gene_name": "Ectonucleotide pyrophosphatase_phosphodiesterase family member 1",
  "term_label": "regulation of bone mineralization",
  "term_id": "GO:0030500"
}